maternal placenta development [GO:0001893] (biological process) Definition: Maternally driven process whose specific outcome is the progression of the placenta over time, from its formation to the mature structure. The placenta is an organ of metabolic interchange between fetus and mother, partly of embryonic origin and partly of maternal origin. Sources: GOC:add, ISBN:068340007X Also known as: decidua development Relationships: is a type of developmental process involved in reproduction [GO:0003006]; is a type of anatomical structure development [GO:0048856]; is a type of maternal process involved in female pregnancy [GO:0060135]; is part of placenta development [GO:0001890]